{
  "term_id": "GO:0005829",
  "gene": "UniProtKB:Q96DR4",
  "gene_name": "StAR-related lipid transfer protein 4",
  "gene_symbol": "STARD4",
  "term_label": "cytosol"
}